positive regulation of vasoconstriction [GO:0045907] (biological process) Definition: Any process that activates or increases the frequency, rate or extent of vasoconstriction. Sources: GOC:go_curators Also known as: up regulation of vasoconstriction, up-regulation of vasoconstriction, upregulation of vasoconstriction, activation of vasoconstriction, stimulation of vasoconstriction Relationships: is a type of regulation of vasoconstriction [GO:0019229]; is_a positive regulation of multicellular organismal process [GO:0051240]; positively regulates vasoconstriction [GO:0042310] Subtypes: positive regulation of vascular associated smooth muscle contraction [GO:1904695]